alveolar secondary septum development [GO:0061144] (biological process) Relationships: is a type of lung epithelium development [GO:0060428]; is part of lung saccule development [GO:0060430] Definition: The progression of a secondary alveolar septum over time, from its formation to the mature structure. A secondary alveolar septum is a specialized epithelium that subdivides the initial saccule. Sources: GOC:dph